{
  "gene": "UniProtKB:Q86SZ2",
  "term_label": "cis-Golgi network",
  "term_id": "GO:0005801",
  "gene_name": "Trafficking protein particle complex subunit 6B",
  "gene_symbol": "TRAPPC6B"
}